{
  "gene_name": "Mothers against decapentaplegic homolog 3",
  "gene": "UniProtKB:P84022",
  "gene_symbol": "SMAD3",
  "term_id": "GO:0032924",
  "term_label": "activin receptor signaling pathway"
}